{
  "gene_name": "E3 ubiquitin-protein ligase MARCHF11",
  "gene": "UniProtKB:A6NNE9",
  "gene_symbol": "MARCHF11",
  "term_id": "UNKNOWN:0002",
  "term_label": "Unknown biological process"
}